negative regulation of zoospore formation [GO:0075242] (BP) Sources: GOC:pamgo_curators Definition: Any process that stops, prevents, or reduces the frequency, rate or extent of zoospore formation, a process in which a diploid cell undergoes meiosis, and the meiotic products acquire specialized features of asexual motile mononucleate flagellated spores called zoospores. Relationships: is a type of regulation of zoospore formation [GO:0075240]; is a type of GO:0075288; negatively regulates zoospore formation [GO:0075239]